IgA B cell receptor complex [GO:0071747] (cellular component) Definition: An IgA immunoglobulin complex that is present in the plasma membrane of B cells and is composed of two identical immunoglobulin heavy chains of an IgA isotype and two identical immunoglobulin light chains and a signaling subunit, a heterodimer of the Ig-alpha and Ig-beta proteins. References: PMID:16362985 Sources: GOC:add, ISBN:0781765196 Note: Note that an IgA immunoglobulin complex has the function of antigen binding if a suitable antigen is available. Also known as: membrane-bound IgA, membrane-bound IgA1, membrane-bound IgA2, surface IgA, surface IgA1, surface IgA2 Relationships: is a type of B cell receptor complex [GO:0019815]; is a type of IgA immunoglobulin complex [GO:0071745]